learning [GO:0007612] (biological process) Sources: ISBN:0582227089, ISBN:0721662544 Subtypes: GO:0008306, GO:0035106, GO:0046958, GO:0061743, observational learning [GO:0098597] Relationships: is a type of GO:0007611 Definition: Any process in an organism in which a relatively long-lasting adaptive behavioral change occurs as the result of experience.